{
  "gene": "UniProtKB:P68032",
  "term_id": "GO:0005884",
  "gene_symbol": "ACTC1",
  "term_label": "actin filament",
  "gene_name": "Actin, alpha cardiac muscle 1"
}